{
  "term_label": "Unknown cellular component",
  "gene_symbol": "ENDOU",
  "gene": "UniProtKB:P21128",
  "gene_name": "Uridylate-specific endoribonuclease",
  "term_id": "UNKNOWN:0003"
}